{
  "term_id": "UNKNOWN:0002",
  "gene_symbol": "MROH2B",
  "gene_name": "Maestro heat-like repeat-containing protein family member 2B",
  "gene": "UniProtKB:Q7Z745",
  "term_label": "Unknown biological process"
}